growth of a germarium-derived egg chamber [GO:0007295] (biological process) Sources: GOC:mtg_sensu, ISBN:0879694238 Also known as: egg chamber growth Relationships: is a type of developmental process involved in reproduction [GO:0003006]; is a type of developmental growth [GO:0048589]; is part of oogenesis [GO:0048477] Definition: Growth of the egg chamber between the time it leaves the germarium and the onset of vitellogenesis. During this time both nurse cells and the oocyte undergo developmental changes including nuclear organization and cytoplasmic growth. An example of this is found in Drosophila melanogaster.